{
  "term_label": "Unknown molecular function",
  "gene_symbol": "HDHD3",
  "term_id": "UNKNOWN:0001",
  "gene_name": "Haloacid dehalogenase-like hydrolase domain-containing protein 3",
  "gene": "UniProtKB:Q9BSH5"
}